{
  "gene_name": "Dicarboxylate carrier SLC25A8",
  "term_label": "adaptive thermogenesis",
  "gene": "UniProtKB:P55851",
  "gene_symbol": "UCP2",
  "term_id": "GO:1990845"
}